glucuronate metabolic process [GO:0019585] (biological process) Relationships: is a type of monocarboxylic acid metabolic process [GO:0032787] Sources: GOC:go_curators, ISBN:0198506732 Subtypes: GO:0006064, GO:0046399 Definition: The chemical reactions and pathways involving glucuronate, any salt or ester of glucuronic acid, the uronic acid formally derived from glucose by oxidation of the hydroxymethylene group at C-6 to a carboxyl group. Also known as: glucuronate metabolism